cellular response to diamide [GO:0072738] (biological process) Sources: GOC:mah Definition: Any process that results in a change in state or activity of a cell (in terms of movement, secretion, enzyme production, gene expression, etc.) as a result of a diamide (N,N,N',N'-tetramethyldiazene-1,2-dicarboxamide) stimulus. Also known as: cellular response to N,N,N',N'-tetramethyldiazene-1,2-dicarboxamide Relationships: is a type of response to diamide [GO:0072737]; is a type of cellular response to nitrogen compound [GO:1901699]